{
  "gene": "UniProtKB:P17483",
  "term_id": "GO:0009952",
  "gene_name": "Homeobox protein Hox-B4",
  "gene_symbol": "HOXB4",
  "term_label": "anterior/posterior pattern specification"
}